aryl hydrocarbon receptor binding [GO:0017162] (molecular function) Relationships: is a type of signaling receptor binding [GO:0005102]; is a type of GO:0061629 Definition: Binding to an aryl hydrocarbon receptor. Sources: GOC:ai